DDEL sequence binding [GO:0030944] (molecular function) Sources: GOC:mah Relationships: is a type of ER retention sequence binding [GO:0046923] Definition: Binding to a KDEL sequence, the C terminus tetrapeptide sequence Asp-Asp-Glu-Leu found in proteins that are to be retained in the endoplasmic reticulum.